{
  "gene_name": "Interferon regulatory factor 2-binding protein 1",
  "term_label": "regulation of transcription by RNA polymerase II",
  "gene": "UniProtKB:Q8IU81",
  "term_id": "GO:0006357",
  "gene_symbol": "IRF2BP1"
}